{
  "gene_symbol": "HTR1F",
  "gene": "UniProtKB:P30939",
  "term_label": "plasma membrane",
  "term_id": "GO:0005886",
  "gene_name": "5-hydroxytryptamine receptor 1F"
}